{
  "gene_symbol": "HLA-DQB2",
  "gene": "UniProtKB:P05538",
  "gene_name": "HLA class II histocompatibility antigen, DQ beta 2 chain",
  "term_id": "GO:0042605",
  "term_label": "peptide antigen binding"
}